clathrin complex [GO:0071439] (cellular component) Also known as: clathrin triskelion Relationships: is a type of membrane protein complex [GO:0098796]; is part of clathrin coat [GO:0030118] Definition: A protein complex that consists of three clathrin heavy chains and three clathrin light chains, organized into a symmetrical three-legged structure called a triskelion. In clathrin-coated vesicles clathrin is the main component of the coat and forms a polymeric mechanical scaffold on the vesicle surface. References: PMID:16493411 Sources: GOC:mah